{
  "gene": "UniProtKB:Q5K4L6",
  "term_id": "GO:0004467",
  "gene_symbol": "SLC27A3",
  "gene_name": "Long-chain fatty acid transport protein 3",
  "term_label": "long-chain fatty acid-CoA ligase activity"
}